{
  "term_label": "plasma membrane",
  "gene": "UniProtKB:Q9HCM2",
  "gene_name": "Plexin-A4",
  "gene_symbol": "PLXNA4",
  "term_id": "GO:0005886"
}